{
  "gene_name": "Urea transporter 2",
  "term_label": "Unknown molecular function",
  "gene": "UniProtKB:Q15849",
  "gene_symbol": "SLC14A2",
  "term_id": "UNKNOWN:0001"
}